misfolded protein transport [GO:0070843] (biological process) Relationships: is a type of intracellular protein transport [GO:0006886] References: PMID:14675537 Sources: GOC:BHF, GOC:mah Definition: The directed movement of misfolded proteins in a cell, including the movement of proteins between specific compartments or structures within a cell. Subtypes: GO:0070845